cellular response to human chorionic gonadotropin stimulus [GO:0044751] (BP) Definition: Any process that results in a change in state or activity of a cell (in terms of movement, secretion, enzyme production, gene expression, etc.) as a result of a human chorionic gonadotropin stimulus. Relationships: is a type of response to human chorionic gonadotropin [GO:0044752]; is_a cellular response to gonadotropin stimulus [GO:0071371] References: PMID:21325635 Also known as: cellular response to human chorionic gonadotrophin stimulus